{
  "gene_symbol": "ADARB2",
  "term_label": "cytoplasm",
  "gene": "UniProtKB:Q9NS39",
  "gene_name": "Double-stranded RNA-specific editase B2",
  "term_id": "GO:0005737"
}